{
  "term_label": "DNA binding",
  "gene": "UniProtKB:O75531",
  "gene_symbol": "BANF1",
  "gene_name": "Barrier-to-autointegration factor",
  "term_id": "GO:0003677"
}